protein transport out of plasma membrane raft [GO:0044862] (biological process) Sources: GOC:jl Definition: The directed movement of a protein out of a plasma membrane raft. Relationships: is a type of protein transport out of membrane raft [GO:0032599]; is a type of protein localization to membrane [GO:0072657]; is a type of establishment of protein localization to membrane [GO:0090150]; is a type of protein transport within plasma membrane [GO:0099632]; is a type of GO:1990778